antigen binding [GO:0003823] (molecular function) Sources: GOC:jl, ISBN:0198506732, ISBN:0721662544 Also known as: B cell receptor activity, MHC activity, major histocompatibility complex activity, major histocompatibility complex antigen display activity, opsonin activity, antibody activity Definition: Binding to an antigen, any substance which is capable of inducing a specific immune response and of reacting with the products of that response, the specific antibody or specifically sensitized T-lymphocytes, or both. Binding may counteract the biological activity of the antigen. Antigen binding by an MHC protein complex allows the antigen to be displayed to a T cell or NK cell. Subtypes: GO:0030882, peptide antigen binding [GO:0042605], GO:1990405 Relationships: is a type of binding [GO:0005488]